{
  "term_id": "UNKNOWN:0001",
  "gene_symbol": "PHLDB3",
  "gene_name": "Pleckstrin homology-like domain family B member 3",
  "gene": "UniProtKB:Q6NSJ2",
  "term_label": "Unknown molecular function"
}